{
  "gene_symbol": "FOXE1",
  "gene_name": "Forkhead box protein E1",
  "gene": "UniProtKB:O00358",
  "term_label": "regulation of transcription by RNA polymerase II",
  "term_id": "GO:0006357"
}